{
  "gene": "UniProtKB:P13349",
  "gene_name": "Myogenic factor 5",
  "gene_symbol": "MYF5",
  "term_id": "GO:0045663",
  "term_label": "positive regulation of myoblast differentiation"
}